regulation of transcription initiation by RNA polymerase I [GO:1903357] (biological process) References: PMID:9092673 Sources: GOC:TermGenie, GO_REF:0000058 Relationships: is a type of regulation of transcription by RNA polymerase I [GO:0006356]; is a type of GO:2000142; regulates GO:0006361 Also known as: regulation of transcription initiation from RNA polymerase I promoter, regulation of transcription initiation from RNA polymerase I promoter for nuclear large rRNA transcript Definition: Any process that modulates the frequency, rate or extent of transcription initiation from RNA polymerase I promoter.